{
  "term_id": "GO:0008395",
  "term_label": "steroid hydroxylase activity",
  "gene": "UniProtKB:O95992",
  "gene_symbol": "CH25H",
  "gene_name": "Cholesterol 25-hydroxylase"
}